positive regulation of interleukin-6-mediated signaling pathway [GO:0070105] (biological process) Relationships: is a type of positive regulation of cytokine-mediated signaling pathway [GO:0001961]; is a type of GO:0070103; positively regulates interleukin-6-mediated signaling pathway [GO:0070102] Definition: Any process that increases the rate, frequency or extent of an interleukin-6-mediated signaling pathway. Also known as: positive regulation of IL-6-mediated signaling pathway, positive regulation of interleukin-6-mediated signalling pathway Sources: GOC:BHF, GOC:mah